{
  "gene_name": "Pyridoxal phosphate phosphatase PHOSPHO2",
  "gene": "UniProtKB:Q8TCD6",
  "gene_symbol": "PHOSPHO2",
  "term_id": "UNKNOWN:0002",
  "term_label": "Unknown biological process"
}